high-affinity thiamine:proton symporter activity [GO:0034216] (molecular function) Also known as: high affinity thiamin:hydrogen symporter activity, high-affinity thiamin:hydrogen symporter activity, high-affinity thiamin:proton symporter activity, high-affinity thiamine:hydrogen symporter activity Relationships: is a type of thiamine:proton symporter activity [GO:0034215] Definition: Enables the transfer of a solute or solutes from one side of a membrane to the other according to the reaction: thiamine(out) + H+(out) = thiamine(in) + H+(in). In high-affinity transport the transporter is able to bind the solute even if it is only present at very low concentrations. Sources: GOC:mah